{
  "term_label": "voltage-gated potassium channel activity",
  "gene_symbol": "KCNH8",
  "term_id": "GO:0005249",
  "gene": "UniProtKB:Q96L42",
  "gene_name": "Potassium voltage-gated channel subfamily H member 8"
}